{
  "term_label": "negative regulation of fibroblast growth factor receptor signaling pathway",
  "gene_name": "Protein sprouty homolog 2",
  "gene_symbol": "SPRY2",
  "gene": "UniProtKB:O43597",
  "term_id": "GO:0040037"
}